{
  "gene_symbol": "NTRK2",
  "term_id": "GO:0048403",
  "gene": "UniProtKB:Q16620",
  "term_label": "brain-derived neurotrophic factor binding",
  "gene_name": "BDNF_NT-3 growth factors receptor"
}